regulation of tumor necrosis factor superfamily cytokine production [GO:1903555] (biological process) References: PMID:24187568 Sources: GOC:TermGenie, GO_REF:0000058 Subtypes: regulation of TRAIL production [GO:0032679], regulation of tumor necrosis factor production [GO:0032680], GO:0032681, negative regulation of tumor necrosis factor superfamily cytokine production [GO:1903556], GO:1903557, regulation of tumor necrosis factor (ligand) superfamily member 11 production [GO:2000307] Relationships: is a type of GO:0001817; regulates tumor necrosis factor superfamily cytokine production [GO:0071706] Also known as: regulation of TNFSF cytokine production, regulation of TNF superfamily production Definition: Any process that modulates the frequency, rate or extent of tumor necrosis factor superfamily cytokine production.